{
  "term_id": "UNKNOWN:0002",
  "gene_name": "Uncharacterized protein",
  "gene_symbol": "A0A8V8TPC4",
  "gene": "UniProtKB:A0A8V8TPC4",
  "term_label": "Unknown biological process"
}